positive T cell selection [GO:0043368] (biological process) References: PMID:12414722 Sources: ISBN:0781735149 Subtypes: positive thymic T cell selection [GO:0045059], GO:0045067 Also known as: positive T lymphocyte selection, positive T-cell selection, positive T-lymphocyte selection Definition: The process of sparing immature T cells which react with self-MHC protein complexes with low affinity levels from apoptotic death. Relationships: is a type of T cell selection [GO:0045058]